{
  "term_id": "GO:0048255",
  "term_label": "mRNA stabilization",
  "gene_symbol": "TENT5C",
  "gene": "UniProtKB:Q5VWP2",
  "gene_name": "Terminal nucleotidyltransferase 5C"
}